{
  "gene_symbol": "HDX",
  "gene": "UniProtKB:Q7Z353",
  "term_label": "DNA-binding transcription factor activity, RNA polymerase II-specific",
  "gene_name": "Highly divergent homeobox",
  "term_id": "GO:0000981"
}